{
  "gene_name": "Sentrin-specific protease 8",
  "term_label": "Unknown cellular component",
  "term_id": "UNKNOWN:0003",
  "gene_symbol": "SENP8",
  "gene": "UniProtKB:Q96LD8"
}